N-cyclopropylammeline deaminase activity [GO:0034548] (molecular function) Sources: UM-BBD_reactionID:r0826 Relationships: is a type of GO:0016814 Definition: Catalysis of the reaction: N-cyclopropylammeline + H2O = N-cyclopropylammelide + NH3.